{
  "term_id": "UNKNOWN:0001",
  "gene": "UniProtKB:Q14624",
  "gene_name": "Inter-alpha-trypsin inhibitor heavy chain H4",
  "term_label": "Unknown molecular function",
  "gene_symbol": "ITIH4"
}